{
  "gene": "UniProtKB:Q14542",
  "gene_name": "Equilibrative nucleoside transporter 2",
  "gene_symbol": "SLC29A2",
  "term_id": "GO:0015853",
  "term_label": "adenine transport"
}